{
  "gene_name": "Ena_VASP-like protein",
  "gene": "UniProtKB:Q9UI08",
  "term_label": "profilin binding",
  "term_id": "GO:0005522",
  "gene_symbol": "EVL"
}